{
  "gene_name": "Small integral membrane protein 43",
  "term_id": "UNKNOWN:0001",
  "gene_symbol": "SMIM43",
  "gene": "UniProtKB:Q4W5P6",
  "term_label": "Unknown molecular function"
}